{
  "term_id": "GO:0032580",
  "gene_symbol": "GOLGA8IP",
  "gene_name": "Putative golgin subfamily A member 8I",
  "term_label": "Golgi cisterna membrane",
  "gene": "UniProtKB:A6NC78"
}